{
  "term_label": "proteolysis",
  "gene_name": "Chymotrypsin-C",
  "term_id": "GO:0006508",
  "gene_symbol": "CTRC",
  "gene": "UniProtKB:Q99895"
}